{
  "gene": "UniProtKB:Q17RS7",
  "gene_symbol": "GEN1",
  "gene_name": "Flap endonuclease GEN homolog 1",
  "term_id": "UNKNOWN:0002",
  "term_label": "Unknown biological process"
}